double membrane vesicle viral factory lumen [GO:0062244] (cellular component) Definition: The volume surrounded by the inner membrane of a double membrane vesicle viral factory. References: PMID:22440839 Also known as: lumen of double membrane vesicle viral factory Relationships: is_a host cell cytoplasm part [GO:0033655]; BFO_0000050 double membrane vesicle viral factory [GO:0039718]